{
  "term_id": "GO:0005730",
  "gene_name": "Unhealthy ribosome biogenesis protein 2 homolog",
  "gene": "UniProtKB:Q14146",
  "gene_symbol": "URB2",
  "term_label": "nucleolus"
}